{
  "term_id": "GO:0006357",
  "term_label": "regulation of transcription by RNA polymerase II",
  "gene": "UniProtKB:A6NN14",
  "gene_name": "Zinc finger protein 729",
  "gene_symbol": "ZNF729"
}